{
  "gene": "UniProtKB:Q75V66",
  "gene_symbol": "ANO5",
  "term_id": "GO:0005886",
  "term_label": "plasma membrane",
  "gene_name": "Anoctamin-5"
}